{
  "gene_name": "DNA-directed RNA polymerase II subunit RPB7",
  "gene_symbol": "POLR2G",
  "term_label": "single-stranded DNA binding",
  "gene": "UniProtKB:P62487",
  "term_id": "GO:0003697"
}